positive regulation of ubiquitin-specific protease activity [GO:2000158] (biological process) Relationships: is a type of positive regulation of peptidase activity [GO:0010952]; positively regulates cysteine-type deubiquitinase activity [GO:0004843] Definition: Any process that activates or increases the frequency, rate or extent of ubiquitin-specific protease (deubiquitinase) activity. Also known as: positive regulation of deubiquitinase activity, positive regulation of ubiquitin hydrolase activity, positive regulation of UBP, positive regulation of UCH2 Sources: GOC:obol